{
  "gene": "UniProtKB:Q13224",
  "gene_name": "Glutamate receptor ionotropic, NMDA 2B",
  "term_label": "plasma membrane",
  "gene_symbol": "GRIN2B",
  "term_id": "GO:0005886"
}